{
  "gene_name": "Smoothelin-like protein 2",
  "term_id": "UNKNOWN:0003",
  "gene": "UniProtKB:Q2TAL5",
  "term_label": "Unknown cellular component",
  "gene_symbol": "SMTNL2"
}